{
  "term_id": "GO:0000978",
  "gene_symbol": "RFX4",
  "term_label": "RNA polymerase II cis-regulatory region sequence-specific DNA binding",
  "gene": "UniProtKB:Q33E94",
  "gene_name": "Transcription factor RFX4"
}